{
  "term_label": "positive regulation of DNA repair",
  "gene_name": "Eyes absent homolog 2",
  "gene_symbol": "EYA2",
  "gene": "UniProtKB:O00167",
  "term_id": "GO:0045739"
}